regulation of actin filament polymerization [GO:0030833] (biological process) Sources: GOC:mah Also known as: regulation of actin polymerization Subtypes: negative regulation of actin filament polymerization [GO:0030837], positive regulation of actin filament polymerization [GO:0030838], regulation of barbed-end actin filament capping [GO:2000812] Definition: Any process that modulates the frequency, rate or extent of the assembly of actin filaments by the addition of actin monomers to a filament. Relationships: is a type of GO:0008064; is a type of GO:0032271; regulates actin filament polymerization [GO:0030041]